Cul4B-RING E3 ubiquitin ligase complex [GO:0031465] (cellular component) Definition: A ubiquitin ligase complex in which a cullin from the Cul4B subfamily and a RING domain protein form the catalytic core; substrate specificity is conferred by unknown subunits. References: PMID:15571813, PMID:15688063 Also known as: cullin-RING ligase 4B Relationships: is_a Cul4-RING E3 ubiquitin ligase complex [GO:0080008]